glucosylglycerol transmembrane transporter activity [GO:0051474] (molecular function) Sources: GOC:ai, GOC:mtg_transport, ISBN:0815340729 Definition: Enables the transfer of a glucosylglycerol from one side of a membrane to the other. A glucosylglycerol is an alpha-D-glucopyranosyl-alpha-(1,2)-glycerol. Relationships: is a type of GO:0015144; is a type of polyol transmembrane transporter activity [GO:0015166]; is a type of carbohydrate derivative transmembrane transporter activity [GO:1901505]; is part of glucosylglycerol transmembrane transport [GO:0051475]